etioplast prolamellar body [GO:0009541] (cellular component) Sources: ISBN:0140514031 Relationships: is_a cellular anatomical structure [GO:0110165]; is part of GO:0009513 Definition: A three dimensional regular lattice found in etioplasts. It is composed of a continuous system of tubules but when exposed to light the symmetrical arrangement is rapidly lost as tubules become pinched off into two dimensional sections of lattice. These for perforated sheets of membrane that move apart, extend and increase, finally establishing the typical granal and intergranal lamellae of the mature chloroplast.